{
  "term_label": "nucleus",
  "term_id": "GO:0005634",
  "gene_name": "Forkhead box protein P3",
  "gene_symbol": "FOXP3",
  "gene": "UniProtKB:Q9BZS1"
}